{
  "gene_symbol": "SYNDIG1L",
  "term_label": "Unknown molecular function",
  "gene": "UniProtKB:A6NDD5",
  "gene_name": "Synapse differentiation-inducing gene protein 1-like",
  "term_id": "UNKNOWN:0001"
}